bI4 intron splicing complex [GO:0106391] (cellular component) Definition: A protein complex required for the splicing of intron 4 of the cytochrome b (COB) gene. In S. cerevisiae, the complex contains the maturase bI4 (which derives from one of the products of the splicing), Leucyl-tRNA synthetase NAM2 and the intron 4 of the cytochrome b pre-mRNA. The two proteins stimulate the ribozyme activity of the pre-mRNA which autoctalyse a group I intron splicing. Relationships: is a type of endoribonuclease complex [GO:1902555] References: PMID:19622748 Sources: GOC:lnp